{
  "term_id": "GO:0000978",
  "gene_name": "Transcription cofactor HES-6",
  "gene": "UniProtKB:Q96HZ4",
  "gene_symbol": "HES6",
  "term_label": "RNA polymerase II cis-regulatory region sequence-specific DNA binding"
}